{
  "term_label": "synaptic transmission, GABAergic",
  "gene_name": "Gamma-aminobutyric acid receptor subunit alpha-5",
  "gene": "UniProtKB:P31644",
  "term_id": "GO:0051932",
  "gene_symbol": "GABRA5"
}